{
  "gene_symbol": "SLCO1A2",
  "term_label": "bile acid transmembrane transporter activity",
  "gene_name": "Solute carrier organic anion transporter family member 1A2",
  "gene": "UniProtKB:P46721",
  "term_id": "GO:0015125"
}